symbiont-mediated perturbation of host actin cytoskeleton via inhibition of actin polymerization [GO:0141034] (biological process) Relationships: is a type of GO:0141027 Definition: The process in which an organism effects a change that disrupts the host actin cytoskeleton by inhibiting host actin from polymerizing. The host is defined as the larger of the organisms involved in a symbiotic interaction. Also known as: perturbation by symbiont of host actin cytoskeleton via inhibition of actin polymerization References: PMID:23409096, PMID:24253566, PMID:30297616